{
  "gene": "UniProtKB:O43586",
  "gene_symbol": "PSTPIP1",
  "term_id": "UNKNOWN:0002",
  "term_label": "Unknown biological process",
  "gene_name": "Proline-serine-threonine phosphatase-interacting protein 1"
}